{
  "gene_symbol": "SLC16A14",
  "term_id": "GO:0008028",
  "term_label": "monocarboxylic acid transmembrane transporter activity",
  "gene_name": "Monocarboxylate transporter 14",
  "gene": "UniProtKB:Q7RTX9"
}